{
  "term_label": "cGMP binding",
  "term_id": "GO:0030553",
  "gene_name": "cGMP-gated cation channel alpha-1",
  "gene_symbol": "CNGA1",
  "gene": "UniProtKB:P29973"
}